{
  "gene_name": "Poly(A)-specific ribonuclease PNLDC1",
  "term_id": "GO:0005783",
  "gene": "UniProtKB:Q8NA58",
  "term_label": "endoplasmic reticulum",
  "gene_symbol": "PNLDC1"
}